Mei2 nuclear dot complex [GO:0033620] (CC) Definition: A ribonucleoprotein complex that forms during meiotic prophase in a fixed position in the horsetail nucleus; contains Mei2 and meiRNA. May play a role in the progression of meiosis I. References: PMID:12808043 Sources: GOC:vw Also known as: Mei2 nuclear dot, Mei2 dot, nuclear body Relationships: is a type of nuclear protein-containing complex [GO:0140513]; is a type of GO:1990904